raffinose:proton symporter activity [GO:0015529] (molecular function) Sources: TC:2.A.1.5.2 Definition: Enables the transfer of a solute or solutes from one side of a membrane to the other according to the reaction: raffinose(out) + H+(out) = raffinose(in) + H+(in). Also known as: raffinose:hydrogen symporter activity Relationships: is a type of carbohydrate:proton symporter activity [GO:0005351]; is_a raffinose transmembrane transporter activity [GO:0015158]